berberine reductase activity [GO:0050623] (MF) Sources: EC:1.5.1.31, RHEA:21268 Also known as: (R)-canadine synthase activity, (R)-tetrahydroberberine:NADP+ oxidoreductase activity Relationships: is a type of GO:0016646 Definition: Catalysis of the reaction: (R)-canadine + 2 NADP+ = berberine + H+ + 2 NADPH.